[ribulose-bisphosphate carboxylase]-lysine N-methyltransferase activity [GO:0030785] (molecular function) Also known as: RuBisCO LSMT activity, RuBisCO methyltransferase activity, S-adenosyl-L-methionine:3-phospho-D-glycerate-carboxy-lyase (dimerizing)-lysine 6-N-methyltransferase activity, S-adenosyl-L-methionine:3-phospho-D-glycerate-carboxy-lyase (dimerizing)-lysine N6-methyltransferase activity, ribulose-1,5-bisphosphate carboxylase/oxygenase large subunit epsilonN-methyltransferase activity, ribulose-bisphosphate carboxylase-lysine N-methyltransferase activity, ribulose-bisphosphate-carboxylase/oxygenase N-methyltransferase activity Definition: Catalysis of the reaction: S-adenosyl-L-methionine + [ribulose-1,5-bisphosphate carboxylase]-lysine = S-adenosyl-L-homocysteine + [ribulose-1,5-bisphosphate carboxylase]-N6-methyl-L-lysine. Sources: EC:2.1.1.127 Relationships: is_a S-adenosylmethionine-dependent methyltransferase activity [GO:0008757]